negative regulation of xylan catabolic process [GO:2001001] (biological process) Definition: Any process that stops, prevents or reduces the frequency, rate or extent of xylan catabolic process. Sources: GOC:mengo_curators Also known as: negative regulation of xylan breakdown, negative regulation of xylan catabolism, negative regulation of xylan degradation Relationships: is a type of negative regulation of hemicellulose catabolic process [GO:2000989]; is a type of regulation of xylan catabolic process [GO:2001000]; RO_0002212 GO:0045493 Subtypes: negative regulation of glucuronoxylan catabolic process [GO:2000916], negative regulation of arabinoxylan-containing compound catabolic process [GO:2000922]